positive regulation of response to furfural [GO:1901444] (biological process) Definition: Any process that activates or increases the frequency, rate or extent of response to furfural. Also known as: up regulation of response to furfural, up-regulation of response to furfural, upregulation of response to furfural, activation of response to furfural Relationships: is a type of positive regulation of response to stimulus [GO:0048584]; is a type of GO:1901442; positively regulates response to furfural [GO:1901426] Sources: GOC:TermGenie, GOC:mengo_curators